{
  "gene_symbol": "RAF1",
  "gene_name": "RAF proto-oncogene serine_threonine-protein kinase",
  "term_label": "mitochondrion",
  "gene": "UniProtKB:P04049",
  "term_id": "GO:0005739"
}